{
  "term_id": "GO:0086005",
  "gene": "UniProtKB:Q9Y6H6",
  "gene_name": "Potassium voltage-gated channel subfamily E member 3",
  "term_label": "ventricular cardiac muscle cell action potential",
  "gene_symbol": "KCNE3"
}